[protein]-3-O-(N-acetyl-D-glucosaminyl)-L-serine/L-threonine O-N-acetyl-alpha-D-glucosaminase activity [GO:0102571] (molecular function) Relationships: is a type of hydrolase activity, hydrolyzing O-glycosyl compounds [GO:0004553]; is a type of catalytic activity, acting on a protein [GO:0140096] Definition: Catalysis of the reaction: 3-O-(N-acetyl-beta-D-glucosaminyl)-L-seryl/L-threonyl-[protein] + H2O = L-seryl//L-threonyl-[protein] + N-acetyl-D-glucosamine. Sources: EC:3.2.1.169